{
  "term_id": "GO:0000209",
  "gene_symbol": "UBE2G1",
  "term_label": "protein polyubiquitination",
  "gene_name": "Ubiquitin-conjugating enzyme E2 G1",
  "gene": "UniProtKB:P62253"
}